extracellular matrix structural constituent conferring tensile strength [GO:0030020] (molecular function) Sources: GOC:mah, ISBN:0815316194 Also known as: core extracellular matrix, core matrisome Note: Extracellular matrix collagen proteins may be annotated to this term. PMID:29632050, PMID:24443019 Definition: A constituent of the extracellular matrix that enables the matrix to resist longitudinal stress. Relationships: is a type of extracellular matrix structural constituent [GO:0005201]